inferior olivary nucleus development [GO:0021713] (biological process) Relationships: is a type of neural nucleus development [GO:0048857]; is part of GO:0021550 Definition: The process whose specific outcome is the progression of the inferior olivary nucleus over time, from its formation to the mature structure. The inferior olivary nucleus is a capsule-shaped structure in the ventral medulla located just lateral and dorsal to the medullary pyramids. Neurons in the inferior olivary nucleus are the source of climbing fiber input to the cerebellar cortex; these neurons have been implicated in various functions, such as learning and timing of movements. Sources: GOC:cls, GOC:dgh, GOC:dph, GOC:jid, GO_REF:0000021 Also known as: inferior olive development